small conductance calcium-activated potassium channel activity [GO:0016286] (molecular function) Definition: Enables the transmembrane transfer of potassium by a channel with a unit conductance of 2 to 20 picoSiemens that opens in response to stimulus by internal calcium ions. Small conductance calcium-activated potassium channels are more sensitive to calcium than are large conductance calcium-activated potassium channels. Transport by a channel involves catalysis of facilitated diffusion of a solute (by an energy-independent process) involving passage through a transmembrane aqueous pore or channel, without evidence for a carrier-mediated mechanism. Also known as: SK KCa channels, SK calcium-activated potassium channel activity, small conductance KCa channels Regulation: negatively regulated by small conductance calcium-activated potassium channel inhibitor activity [GO:0140629] Relationships: is a type of GO:0015269 Sources: GOC:mtg_transport, OMIM:602754